{
  "gene_symbol": "GNB3",
  "term_label": "G protein-coupled receptor signaling pathway",
  "term_id": "GO:0007186",
  "gene": "UniProtKB:P16520",
  "gene_name": "Guanine nucleotide-binding protein G(I)_G(S)_G(T) subunit beta-3"
}